anaerobic ethylbenzene catabolic process [GO:0010130] (biological process) Also known as: anaerobic ethylbenzene breakdown, anaerobic ethylbenzene catabolism, anaerobic ethylbenzene degradation Relationships: is a type of ethylbenzene catabolic process [GO:0018915] Definition: The chemical reactions and pathways resulting in the breakdown of ethylbenzene, a benzene derivative with an ethyl group attached to the ring, which occurs in the absence of oxygen. Sources: GOC:pz